{
  "gene_name": "N-terminal EF-hand calcium-binding protein 3",
  "gene": "UniProtKB:Q96P71",
  "term_label": "Golgi cis cisterna",
  "term_id": "GO:0000137",
  "gene_symbol": "NECAB3"
}